FHA domain binding [GO:0070975] (molecular function) Sources: GOC:mah, InterPro:IPR000253 Also known as: Forkhead-associated domain binding Definition: Binding to a FHA domain of a protein. The FHA domain is a phosphopeptide recognition domain found in many regulatory proteins, and consists of approximately 80-100 amino acid residues folded into an 11-stranded beta sandwich. Relationships: is a type of protein domain specific binding [GO:0019904]